{
  "gene_symbol": "USP17L8",
  "gene": "UniProtKB:P0C7I0",
  "term_id": "GO:0031647",
  "term_label": "regulation of protein stability",
  "gene_name": "Inactive ubiquitin carboxyl-terminal hydrolase 17-like protein 8"
}